{
  "term_label": "Unknown molecular function",
  "gene_name": "Proline-rich protein 20C",
  "gene_symbol": "PRR20C",
  "gene": "UniProtKB:P86479",
  "term_id": "UNKNOWN:0001"
}